galactomannan biosynthetic process [GO:0051070] (biological process) Relationships: is a type of polysaccharide biosynthetic process [GO:0000271]; is a type of galactomannan metabolic process [GO:0051069] Sources: GOC:ai Also known as: galactomannan anabolism, galactomannan biosynthesis, galactomannan formation, galactomannan synthesis Definition: The chemical reactions and pathways resulting in the formation of galactomannan, a polysaccharide composed of D-galactosyl and D-mannosyl. The mannosyl units form the backbone structure (a linear main chain) with the D-galactosyl as single side units.